myo-inositol hexakisphosphate biosynthetic process, lipid-dependent [GO:0033545] (biological process) Relationships: is a type of myo-inositol hexakisphosphate biosynthetic process [GO:0010264] Definition: The chemical reactions and pathways resulting in the formation of 1D-myo-inositol 1,2,3,4,5,6-hexakisphosphate, phytate, by a pathway using inositol 1,4,5-trisphosphate produced from phosphatidylinositol 4,5-biphosphate hydrolysis by phospholipase C. Also known as: myo-inositol hexakisphosphate anabolism, lipid-dependent, myo-inositol hexakisphosphate biosynthesis, lipid-dependent, myo-inositol hexakisphosphate formation, lipid-dependent, myo-inositol hexakisphosphate synthesis, lipid-dependent, phytate biosynthesis, lipid-dependent, phytate biosynthetic process, lipid-dependent Sources: GOC:mah, MetaCyc:PWY-6555 Subtypes: myo-inositol hexakisphosphate biosynthetic process, via inositol 1,3,4-trisphosphate [GO:0033546]